muscle cell differentiation [GO:0042692] (biological process) Also known as: myogenesis Definition: The process in which a relatively unspecialized cell acquires specialized features of a muscle cell. Sources: CL:0000187, GOC:go_curators Subtypes: smooth muscle cell differentiation [GO:0051145], striated muscle cell differentiation [GO:0051146] Regulation: regulated by regulation of muscle cell differentiation [GO:0051147]; negatively regulated by negative regulation of muscle cell differentiation [GO:0051148]; positively regulated by GO:0051149 Relationships: is a type of cell differentiation [GO:0030154]; is part of muscle structure development [GO:0061061]